negative regulation of protein processing involved in protein targeting to mitochondrion [GO:1903217] (biological process) Definition: Any process that stops, prevents or reduces the frequency, rate or extent of protein processing involved in protein targeting to mitochondrion. References: PMID:21370995 Sources: GOC:PARL, GOC:TermGenie, GOC:bf, GO_REF:0000058 Also known as: down regulation of protein processing involved in protein targeting to mitochondrion, down-regulation of protein processing involved in protein targeting to mitochondrion, downregulation of protein processing involved in protein targeting to mitochondrion, inhibition of protein processing involved in protein targeting to mitochondrion, down regulation of mitochondrial protein processing during import, down-regulation of mitochondrial protein processing during import, downregulation of mitochondrial protein processing during import, inhibition of mitochondrial protein processing during import, negative regulation of mitochondrial protein processing during import Relationships: is a type of negative regulation of protein processing [GO:0010955]; is a type of regulation of protein processing involved in protein targeting to mitochondrion [GO:1903216]; negatively regulates protein processing involved in protein targeting to mitochondrion [GO:0006627]